transposable element silencing by mRNA destabilization [GO:0141008] (biological process) Definition: A transposable element silencing mechanism in which mRNAs transcribed from transposons are targeted for degradation. Sources: GOC:curators Also known as: post-transcriptional retrotransposon silencing, retrotransposon silencing by mRNA destabilization Relationships: is_a GO:0010526; is a type of mRNA destabilization [GO:0061157] Subtypes: GO:0141009, GO:0141011